protein-phosphocysteine-mannitol phosphotransferase system transporter activity [GO:0090565] (molecular function) Relationships: is a type of protein-phosphocysteine-sugar phosphotransferase activity [GO:0090563] Definition: Catalysis of the PEP-dependent, phosphoryl transfer-driven transport of substances across a membrane. The transport happens by catalysis of the reaction: protein S-phosphocysteine + mannitol(out) = protein cysteine + mannitol phosphate(in). This differs from primary and secondary active transport in that the solute is modified during transport. Sources: GOC:am